{
  "term_label": "regulation of transcription by RNA polymerase II",
  "term_id": "GO:0006357",
  "gene_symbol": "ETV6",
  "gene": "UniProtKB:P41212",
  "gene_name": "Transcription factor ETV6"
}